immune response [GO:0006955] (biological process) Sources: GOC:add, GO_REF:0000022 Subtypes: adaptive immune response [GO:0002250], GO:0002251, immune response in gut-associated lymphoid tissue [GO:0002387], immune response to tumor cell [GO:0002418], inflammatory response to antigenic stimulus [GO:0002437], GO:0006959, type 2 immune response [GO:0042092], innate immune response [GO:0045087], immune response involved in response to exogenous dsRNA [GO:1902615] Relationships: is a type of immune system process [GO:0002376]; is a type of response to stimulus [GO:0050896] Regulation: regulated by regulation of immune response [GO:0050776]; negatively regulated by negative regulation of immune response [GO:0050777]; positively regulated by positive regulation of immune response [GO:0050778] Definition: Any immune system process that functions in the calibrated response of an organism to a potential internal or invasive threat.